{
  "gene": "UniProtKB:P00734",
  "gene_name": "Prothrombin",
  "term_label": "extracellular space",
  "term_id": "GO:0005615",
  "gene_symbol": "F2"
}